{
  "gene_name": "Low-density lipoprotein receptor-related protein 11",
  "term_id": "UNKNOWN:0002",
  "term_label": "Unknown biological process",
  "gene": "UniProtKB:Q86VZ4",
  "gene_symbol": "LRP11"
}